{
  "term_id": "GO:0090090",
  "gene_name": "Chromodomain-helicase-DNA-binding protein 8",
  "term_label": "negative regulation of canonical Wnt signaling pathway",
  "gene_symbol": "CHD8",
  "gene": "UniProtKB:Q9HCK8"
}